{
  "gene_symbol": "RAB40A",
  "term_label": "plasma membrane",
  "gene": "UniProtKB:Q8WXH6",
  "gene_name": "Ras-related protein Rab-40A",
  "term_id": "GO:0005886"
}